{
  "term_label": "perinuclear region of cytoplasm",
  "term_id": "GO:0048471",
  "gene": "UniProtKB:Q58FF6",
  "gene_symbol": "HSP90AB4P",
  "gene_name": "Putative heat shock protein HSP 90-beta 4"
}